{
  "term_label": "cytosolic small ribosomal subunit",
  "gene_name": "Small ribosomal subunit protein eS19",
  "term_id": "GO:0022627",
  "gene": "UniProtKB:P39019",
  "gene_symbol": "RPS19"
}